{
  "gene": "UniProtKB:O60688",
  "term_label": "Unknown molecular function",
  "gene_symbol": "YPEL1",
  "gene_name": "Protein yippee-like 1",
  "term_id": "UNKNOWN:0001"
}